{
  "term_id": "GO:0015459",
  "gene_symbol": "KCNG3",
  "term_label": "potassium channel regulator activity",
  "gene": "UniProtKB:Q8TAE7",
  "gene_name": "Potassium voltage-gated channel subfamily G member 3"
}